{
  "gene_symbol": "GRIK4",
  "term_label": "postsynaptic density membrane",
  "term_id": "GO:0098839",
  "gene": "UniProtKB:Q16099",
  "gene_name": "Glutamate receptor ionotropic, kainate 4"
}